retinol transport [GO:0034633] (biological process) Sources: GOC:BHF, GOC:mah, GOC:vk Also known as: vitamin A1 transport Relationships: is a type of organic hydroxy compound transport [GO:0015850]; is a type of terpenoid transport [GO:0046865] Definition: The directed movement of retinol into, out of or within a cell, or between cells, by means of some agent such as a transporter or pore. Retinol is vitamin A1, 2,6,6-trimethyl-1-(9'-hydroxy-3',7'-dimethylnona-1',3',5',7'-tetraenyl)cyclohex-1-ene, one of the three components that makes up vitamin A.